{
  "term_label": "Unknown biological process",
  "gene_name": "Uncharacterized protein C5orf52",
  "gene": "UniProtKB:A6NGY3",
  "gene_symbol": "C5orf52",
  "term_id": "UNKNOWN:0002"
}